{
  "gene_symbol": "ABHD6",
  "term_id": "GO:0046464",
  "gene_name": "Monoacylglycerol lipase ABHD6",
  "term_label": "acylglycerol catabolic process",
  "gene": "UniProtKB:Q9BV23"
}